{
  "term_id": "GO:0005634",
  "gene_name": "LIM_homeobox protein Lhx6",
  "term_label": "nucleus",
  "gene": "UniProtKB:Q9UPM6",
  "gene_symbol": "LHX6"
}